Met1-linked polyubiquitin deubiquitinase activity [GO:0061815] (molecular function) Also known as: deubiquitinase, acting on linear ubiquitin, Met1 linkage specific DUB, cysteine-type deubiquitinase activity, acting on linear ubiquitin, linear ubiquitin specific deubiquitinase activity, ubiquitinyl hydrolase activity, acting on linear ubiquitin Relationships: is a type of cysteine-type deubiquitinase activity [GO:0004843] References: PMID:26503766, PMID:27702987 Sources: GOC:dph Definition: Catalysis of the hydrolysis of ubiquitin units from Met1-linked (or linear) polyubiquitin chains.